{
  "gene": "UniProtKB:Q5TBA9",
  "gene_symbol": "FRY",
  "gene_name": "Protein furry homolog",
  "term_label": "cell morphogenesis",
  "term_id": "GO:0000902"
}